{
  "gene": "UniProtKB:P53804",
  "term_id": "UNKNOWN:0003",
  "term_label": "Unknown cellular component",
  "gene_name": "E3 ubiquitin-protein ligase TTC3",
  "gene_symbol": "TTC3"
}